{
  "term_id": "GO:0015117",
  "gene": "UniProtKB:Q9UBX3",
  "term_label": "thiosulfate transmembrane transporter activity",
  "gene_name": "Mitochondrial dicarboxylate carrier",
  "gene_symbol": "SLC25A10"
}